{
  "gene_symbol": "DNHD1",
  "term_id": "GO:0036156",
  "term_label": "inner dynein arm",
  "gene_name": "Dynein heavy chain domain-containing protein 1",
  "gene": "UniProtKB:Q96M86"
}